{
  "term_label": "Unknown molecular function",
  "gene_name": "Charged multivesicular body protein 3",
  "gene_symbol": "CHMP3",
  "term_id": "UNKNOWN:0001",
  "gene": "UniProtKB:Q9Y3E7"
}